nicotinate catabolic process [GO:1901848] (biological process) Definition: The chemical reactions and pathways resulting in the breakdown of nicotinate. Also known as: nicotinate breakdown, nicotinate catabolism, nicotinate degradation Sources: GOC:TermGenie, GOC:yaf, UniPathway:UPA00830 Relationships: is a type of GO:0009822; is a type of monocarboxylic acid catabolic process [GO:0072329]; is a type of pyridine-containing compound catabolic process [GO:0072526]; is a type of nicotinate metabolic process [GO:1901847]